visual behavior [GO:0007632] (biological process) Relationships: is a type of behavior [GO:0007610]; is a type of response to light stimulus [GO:0009416] Subtypes: pattern orientation [GO:0007633], optokinetic behavior [GO:0007634], visual learning [GO:0008542] Also known as: behavioral response to visual stimulus, behavioural response to visual stimulus, visual behaviour Definition: The behavior of an organism in response to a visual stimulus. Sources: GOC:jid, GOC:pr